{
  "gene_name": "Very-long-chain (3R)-3-hydroxyacyl-CoA dehydratase 3",
  "gene": "UniProtKB:Q9P035",
  "term_id": "GO:0018812",
  "gene_symbol": "HACD3",
  "term_label": "3-hydroxyacyl-CoA dehydratase activity"
}